{
  "gene_symbol": "IL17A",
  "gene_name": "Interleukin-17A",
  "term_label": "Unknown molecular function",
  "term_id": "UNKNOWN:0001",
  "gene": "UniProtKB:Q16552"
}